{
  "term_label": "Unknown cellular component",
  "gene": "UniProtKB:Q9C0B7",
  "gene_symbol": "TANGO6",
  "term_id": "UNKNOWN:0003",
  "gene_name": "Transport and Golgi organization protein 6 homolog"
}